{
  "term_label": "Unknown biological process",
  "gene_symbol": "TPTE2P1",
  "term_id": "UNKNOWN:0002",
  "gene_name": "Putative phosphatidylinositol 3,4,5-trisphosphate 3-phosphatase TPTE2P1",
  "gene": "UniProtKB:Q5T6R2"
}